{
  "gene": "UniProtKB:P43003",
  "gene_name": "Excitatory amino acid transporter 1",
  "term_id": "GO:0005886",
  "gene_symbol": "SLC1A3",
  "term_label": "plasma membrane"
}